{
  "term_label": "hemidesmosome",
  "gene_name": "Dystonin",
  "gene": "UniProtKB:Q03001",
  "term_id": "GO:0030056",
  "gene_symbol": "DST"
}